regulation of protein phosphorylation [GO:0001932] (biological process) Sources: GOC:hjd Subtypes: negative regulation of protein phosphorylation [GO:0001933], positive regulation of protein phosphorylation [GO:0001934], GO:0010799, regulation of eIF2 alpha phosphorylation by heme [GO:0010999], regulation of protein autophosphorylation [GO:0031952], GO:0033135, regulation of protein kinase activity [GO:0045859], GO:0050730, GO:0060734, regulation of eIF2 alpha phosphorylation by dsRNA [GO:0060735], GO:1903719, regulation of inhibitory G protein-coupled receptor phosphorylation [GO:1904323] Relationships: is a type of regulation of protein modification process [GO:0031399]; is a type of regulation of phosphorylation [GO:0042325]; regulates protein phosphorylation [GO:0006468] Also known as: regulation of protein amino acid phosphorylation Definition: Any process that modulates the frequency, rate or extent of addition of phosphate groups into an amino acid in a protein.